molybdate ion binding [GO:0030973] (molecular function) Definition: Binding to a molybdate ion (MoO4 2-). Sources: GOC:mlg Also known as: MoO4 ion binding Relationships: is a type of anion binding [GO:0043168]